histone H4K16 acetyltransferase activity [GO:0046972] (molecular function) References: PMID:18552846, PMID:19056256 Note: Note that the residue position corresponds to the canonical human H4 histone (UniProtKB:P02309); this residue is conserved across all eukaryotes. Note that the initiation methionine is cleaved, so the first residue is S1. Relationships: is a type of histone H4 acetyltransferase activity [GO:0010485] Also known as: histone acetylase activity (H4-K16 specific), histone acetyltransferase activity (H4-K16 specific), histone lysine acetyltransferase activity (H4-K16 specific) Definition: Catalysis of the reaction: acetyl-CoA + histone H4 L-lysine (position 16) = CoA + histone H4 N6-acetyl-L-lysine (position 16). This reaction represents the addition of an acetyl group to the lysine at position 16 of histone H4.